pyrimidine nucleoside interconversion [GO:0019689] (biological process) Sources: GOC:mah, ISBN:0306444747, ISBN:0471394831 Subtypes: GO:0019690 Definition: The chemical reactions and pathways by which a pyrimidine nucleoside is synthesized from another pyrimidine nucleoside. Relationships: is a type of pyrimidine nucleoside metabolic process [GO:0006213]; is_a nucleobase-containing small molecule interconversion [GO:0015949]